{
  "gene_symbol": "BFAR",
  "gene_name": "Bifunctional apoptosis regulator",
  "gene": "UniProtKB:Q9NZS9",
  "term_label": "proteasome-mediated ubiquitin-dependent protein catabolic process",
  "term_id": "GO:0043161"
}